{
  "term_id": "UNKNOWN:0002",
  "term_label": "Unknown biological process",
  "gene_name": "Ribosomal oxygenase 2",
  "gene": "UniProtKB:Q8IUF8",
  "gene_symbol": "RIOX2"
}